{
  "gene": "UniProtKB:O96009",
  "term_label": "proteolysis",
  "term_id": "GO:0006508",
  "gene_name": "Napsin-A",
  "gene_symbol": "NAPSA"
}